DiaA complex [GO:1990125] (cellular component) Definition: A homotetrameric protein complex consisting of a symmetrical pair of DiaA homodimers. Facilitates DnaA binding to the origin of replication during replication initiation. References: PMID:17699754 Sources: GOC:bhm Also known as: DiaA homotetramer Relationships: is a type of protein-containing complex [GO:0032991]